integrin alpha11-beta1 complex [GO:0034681] (cellular component) Definition: An integrin complex that comprises one alpha11 subunit and one beta1 subunit. References: PMID:12297042 Also known as: alpha11-beta1 integrin complex, ITGA11-ITGB1 complex Relationships: is a type of integrin complex [GO:0008305]